ADP metabolic process [GO:0046031] (biological process) Definition: The chemical reactions and pathways involving ADP, adenosine 5'-diphosphate. Also known as: ADP metabolism Sources: GOC:go_curators Subtypes: ADP biosynthetic process [GO:0006172], dATP biosynthetic process from ADP [GO:0006176], ADP catabolic process [GO:0046032] Relationships: is_a purine ribonucleotide metabolic process [GO:0009150]; is a type of GO:0009179